{
  "gene_name": "Rho guanine nucleotide exchange factor 25",
  "term_label": "guanyl-nucleotide exchange factor activity",
  "term_id": "GO:0005085",
  "gene": "UniProtKB:Q86VW2",
  "gene_symbol": "ARHGEF25"
}